positive regulation of artery morphogenesis [GO:1905653] (biological process) Subtypes: positive regulation of aorta morphogenesis [GO:1903849], GO:1904337 References: PMID:27389411 Sources: GOC:BHF, GOC:BHF_miRNA, GOC:TermGenie, GOC:rph, GO_REF:0000058 Also known as: positive regulation of arterial morphogenesis, positive regulation of arteriogenesis, up regulation of arterial morphogenesis, up regulation of arteriogenesis, up regulation of artery morphogenesis, up-regulation of arterial morphogenesis, up-regulation of arteriogenesis, up-regulation of artery morphogenesis, upregulation of arterial morphogenesis, upregulation of arteriogenesis, upregulation of artery morphogenesis, activation of arterial morphogenesis, activation of arteriogenesis, activation of artery morphogenesis Definition: Any process that activates or increases the frequency, rate or extent of artery morphogenesis. Relationships: is a type of positive regulation of developmental process [GO:0051094]; is a type of regulation of artery morphogenesis [GO:1905651]; positively regulates artery morphogenesis [GO:0048844]